{
  "term_id": "GO:0006367",
  "term_label": "transcription initiation at RNA polymerase II promoter",
  "gene_symbol": "TAF8",
  "gene": "UniProtKB:Q7Z7C8",
  "gene_name": "Transcription initiation factor TFIID subunit 8"
}